negative regulation of death-inducing signaling complex assembly [GO:1903073] (biological process) Relationships: is_a negative regulation of protein-containing complex assembly [GO:0031333]; is a type of GO:1903072; is a type of negative regulation of extrinsic apoptotic signaling pathway [GO:2001237]; negatively regulates death-inducing signaling complex assembly [GO:0071550] Definition: Any process that stops, prevents or reduces the frequency, rate or extent of death-inducing signaling complex assembly. References: PMID:21785459 Sources: GOC:PARL, GOC:TermGenie, GOC:bf, GO_REF:0000058 Also known as: down regulation of DD-mediated complex assembly, down regulation of DISC assembly, down regulation of DISC formation, down regulation of death domain-mediated complex assembly, down regulation of death domain-mediated complex assembly involved in extrinsic apoptotic pathway, down regulation of death-inducing signaling complex assembly, down regulation of death-inducing signaling complex formation, down regulation of death-inducing signalling complex assembly, down-regulation of DD-mediated complex assembly, down-regulation of DISC assembly, down-regulation of DISC formation, down-regulation of death domain-mediated complex assembly, down-regulation of death domain-mediated complex assembly involved in extrinsic apoptotic pathway, down-regulation of death-inducing signaling complex assembly, down-regulation of death-inducing signaling complex formation, down-regulation of death-inducing signalling complex assembly, downregulation of DD-mediated complex assembly, downregulation of DISC assembly, downregulation of DISC formation, downregulation of death domain-mediated complex assembly, downregulation of death domain-mediated complex assembly involved in extrinsic apoptotic pathway, downregulation of death-inducing signaling complex assembly, downregulation of death-inducing signaling complex formation, downregulation of death-inducing signalling complex assembly, negative regulation of DD-mediated complex assembly, negative regulation of DISC assembly, negative regulation of DISC formation, negative regulation of death domain-mediated complex assembly, negative regulation of death domain-mediated complex assembly involved in extrinsic apoptotic pathway, negative regulation of death-inducing signaling complex formation, negative regulation of death-inducing signalling complex assembly, inhibition of DD-mediated complex assembly, inhibition of DISC assembly, inhibition of DISC formation, inhibition of death domain-mediated complex assembly, inhibition of death domain-mediated complex assembly involved in extrinsic apoptotic pathway, inhibition of death-inducing signaling complex assembly, inhibition of death-inducing signaling complex formation, inhibition of death-inducing signalling complex assembly